{
  "gene_symbol": "ANO9",
  "term_id": "GO:0005886",
  "gene_name": "Anoctamin-9",
  "gene": "UniProtKB:A1A5B4",
  "term_label": "plasma membrane"
}